{
  "term_id": "GO:0045202",
  "gene_symbol": "CHRNA10",
  "gene": "UniProtKB:Q9GZZ6",
  "term_label": "synapse",
  "gene_name": "Neuronal acetylcholine receptor subunit alpha-10"
}